{
  "term_label": "Unknown biological process",
  "gene": "UniProtKB:Q8N2S1",
  "term_id": "UNKNOWN:0002",
  "gene_symbol": "LTBP4",
  "gene_name": "Latent-transforming growth factor beta-binding protein 4"
}